myeloid cell activation involved in immune response [GO:0002275] (biological process) Relationships: is a type of GO:0002274; is a type of leukocyte activation involved in immune response [GO:0002366] Definition: A change in the morphology or behavior of a myeloid cell resulting from exposure to an activating factor such as a cellular or soluble ligand, leading to the initiation or perpetuation of an immune response. Sources: GOC:add, ISBN:0781735149 Subtypes: GO:0002277, eosinophil activation involved in immune response [GO:0002278], GO:0002279, monocyte activation involved in immune response [GO:0002280], neutrophil activation involved in immune response [GO:0002283] Also known as: myeloid cell activation during immune response